{
  "term_id": "GO:0072686",
  "gene": "UniProtKB:Q9Y448",
  "gene_symbol": "KNSTRN",
  "term_label": "mitotic spindle",
  "gene_name": "Small kinetochore-associated protein"
}